nephrostome development [GO:0039018] (biological process) Definition: The process whose specific outcome is the progression of the nephrostome over time, from its formation to the mature structure. The nephrostome is the opening of the pronephros into the body cavity. Relationships: is a type of anatomical structure development [GO:0048856]; is part of GO:0048793 References: PMID:14686690, PMID:15647339 Sources: GOC:mtg_kidney_jan10, XAO:0000062